{
  "gene": "UniProtKB:Q494X3",
  "gene_symbol": "ZNF404",
  "term_id": "GO:0005634",
  "gene_name": "Zinc finger protein 404",
  "term_label": "nucleus"
}